{
  "gene_name": "Probable palmitoyltransferase ZDHHC11B",
  "term_label": "endoplasmic reticulum",
  "gene": "UniProtKB:P0C7U3",
  "gene_symbol": "ZDHHC11B",
  "term_id": "GO:0005783"
}